{
  "gene_symbol": "DNAAF1",
  "gene": "UniProtKB:Q8NEP3",
  "term_id": "GO:0007368",
  "gene_name": "Dynein axonemal assembly factor 1",
  "term_label": "determination of left/right symmetry"
}